{
  "term_label": "transmembrane transporter binding",
  "gene_symbol": "PACS2",
  "term_id": "GO:0044325",
  "gene_name": "Phosphofurin acidic cluster sorting protein 2",
  "gene": "UniProtKB:Q86VP3"
}